{
  "gene_symbol": "OPN5",
  "term_label": "cellular response to light stimulus",
  "term_id": "GO:0071482",
  "gene_name": "Opsin-5",
  "gene": "UniProtKB:Q6U736"
}